{
  "term_id": "GO:0035497",
  "gene_symbol": "CREB3L1",
  "gene_name": "Cyclic AMP-responsive element-binding protein 3-like protein 1",
  "term_label": "cAMP response element binding",
  "gene": "UniProtKB:Q96BA8"
}